{
  "term_id": "GO:0019509",
  "term_label": "L-methionine salvage from methylthioadenosine",
  "gene": "UniProtKB:Q9UHY7",
  "gene_name": "Enolase-phosphatase E1",
  "gene_symbol": "ENOPH1"
}